formate dehydrogenase (NAD+) activity [GO:0008863] (molecular function) Sources: EC:1.17.1.9, RHEA:15985 Relationships: is a type of GO:0016620 Definition: Catalysis of the reaction: formate + NAD+ = CO2 + NADH. Also known as: NAD-dependent formate dehydrogenase, NAD-formate dehydrogenase, formate dehydrogenase (NAD), formate hydrogenlyase, formate-NAD oxidoreductase, formic acid dehydrogenase, formic hydrogen-lyase